{
  "gene_name": "P2Y purinoceptor 6",
  "term_label": "G protein-coupled ADP receptor activity",
  "term_id": "GO:0001621",
  "gene": "UniProtKB:Q15077",
  "gene_symbol": "P2RY6"
}